{
  "gene_symbol": "RBM3",
  "gene_name": "RNA-binding protein 3",
  "term_id": "GO:0003729",
  "term_label": "mRNA binding",
  "gene": "UniProtKB:P98179"
}